neuromuscular junction [GO:0031594] (cellular component) Definition: The junction between the axon of a motor neuron and a muscle fiber. In response to the arrival of action potentials, the presynaptic button releases molecules of neurotransmitters into the synaptic cleft. These diffuse across the cleft and transmit the signal to the postsynaptic membrane of the muscle fiber, leading to a change in post-synaptic potential. Sources: GOC:nln Also known as: NMJ, motor endplate Note: In vertebrates, the term 'neuromuscular junction' is limited to synapses targeting skeletal muscle fibers - all of which are cholinergic and excitatory. Both inhibitory and excitatory neuromuscular junctions exist in invertebrates, utilizing a range of neurotransmitters including glutamate, GABA and 5-HT. Relationships: is a type of synapse [GO:0045202] Subtypes: excitatory neuromuscular junction [GO:0098520], inhibitory neuromuscular junction [GO:0098521], neuromuscular junction of myotube [GO:0098523], neuromuscular junction of somatic muscle [GO:0098527]